{
  "gene_symbol": "TENT4B",
  "gene": "UniProtKB:Q8NDF8",
  "term_label": "TRAMP complex",
  "term_id": "GO:0031499",
  "gene_name": "Terminal nucleotidyltransferase 4B"
}